{
  "gene": "UniProtKB:Q9ULK4",
  "term_label": "positive regulation of gene expression",
  "term_id": "GO:0010628",
  "gene_name": "Mediator of RNA polymerase II transcription subunit 23",
  "gene_symbol": "MED23"
}